squalene synthase [NAD(P)H] activity [GO:0051996] (MF) Relationships: is_a prenyltransferase activity [GO:0004659] Sources: EC:2.5.1.21 Definition: Catalysis of the reaction: 2 (2E,6E)-farnesyl diphosphate + H+ + NAD(P)H = 2 diphosphate + NAD(P)+ + squalene. Also known as: farnesyltransferase activity, presqualene synthase activity, presqualene-diphosphate synthase activity, squalene synthase activity, farnesyl-diphosphate farnesyltransferase activity, squalene synthetase activity